{
  "gene": "UniProtKB:Q6ZWE6",
  "term_label": "Unknown cellular component",
  "gene_name": "Pleckstrin homology domain-containing family M member 3",
  "gene_symbol": "PLEKHM3",
  "term_id": "UNKNOWN:0003"
}